venom-mediated perturbation of mast cell degranulation [GO:0044479] (biological process) Also known as: envenomation resulting in modulation of mast cell degranulation in another organism, envenomation resulting in modulation of mast cell degranulation in other organism References: PMID:21549739 Sources: GOC:fj, GOC:jl Relationships: is a type of venom-mediated perturbation of biological process [GO:0035738] Definition: A process in which an organism alters or subverts mast cell degranulation in another organism via the action of a venom. Subtypes: venom-mediated mast cell degranulation [GO:0044480]